{
  "gene_symbol": "TSLP",
  "gene_name": "Thymic stromal lymphopoietin",
  "term_label": "positive regulation of cytokine-mediated signaling pathway",
  "gene": "UniProtKB:Q969D9",
  "term_id": "GO:0001961"
}